{
  "gene": "UniProtKB:O60513",
  "gene_name": "Beta-1,4-galactosyltransferase 4",
  "gene_symbol": "B4GALT4",
  "term_id": "UNKNOWN:0002",
  "term_label": "Unknown biological process"
}